{
  "gene_name": "Lysine-specific demethylase 2A",
  "term_label": "histone demethylase activity",
  "term_id": "GO:0032452",
  "gene_symbol": "KDM2A",
  "gene": "UniProtKB:Q9Y2K7"
}